{
  "term_id": "GO:0097038",
  "gene_name": "Oxysterol-binding protein-related protein 6",
  "gene_symbol": "OSBPL6",
  "gene": "UniProtKB:Q9BZF3",
  "term_label": "perinuclear endoplasmic reticulum"
}